vascular endothelial growth factor receptor-1 signaling pathway [GO:0036323] (biological process) Sources: GOC:bf, GOC:uh, Wikipedia:FLT1, Wikipedia:VEGF_receptors Definition: The series of molecular signals initiated by a ligand binding to a vascular endothelial growth factor receptor-1 (VEGFR-1) on the surface of a target cell, and ending with the regulation of a downstream cellular process, e.g. transcription. Relationships: is_a GO:0048010 Also known as: FLT1 signaling pathway, VEGFR-1 signaling pathway, VEGFR1 signaling pathway